{
  "gene_name": "Probable E3 ubiquitin-protein ligase HERC1",
  "term_label": "Unknown biological process",
  "gene": "UniProtKB:Q15751",
  "gene_symbol": "HERC1",
  "term_id": "UNKNOWN:0002"
}